{
  "gene_name": "Sodium_hydrogen exchanger 1",
  "term_id": "GO:0071805",
  "gene_symbol": "SLC9A1",
  "gene": "UniProtKB:P19634",
  "term_label": "potassium ion transmembrane transport"
}